calcium export from the mitochondrion involved in positive regulation of presynaptic cytosolic calcium concentration [GO:1905741] (BP) Definition: Any mitochondrial calcium release that is involved in positive regulation of presynaptic cytosolic calcium concentration. References: PMID:26644474 Sources: GOC:TermGenie, GO_REF:0000060 Also known as: calcium ion transmembrane export from mitochondrion involved in positive regulation of presynaptic cytosolic calcium concentration, mitochondrial calcium release involved in positive regulation of presynaptic cytosolic calcium concentration Relationships: is a type of establishment of localization in cell [GO:0051649]; is a type of GO:0099093; is part of positive regulation of presynaptic cytosolic calcium concentration [GO:0099533]